{
  "gene_name": "Zinc finger protein 813",
  "gene": "UniProtKB:Q6ZN06",
  "term_label": "RNA polymerase II cis-regulatory region sequence-specific DNA binding",
  "gene_symbol": "ZNF813",
  "term_id": "GO:0000978"
}